{
  "term_id": "GO:0004126",
  "gene_name": "C-U-editing enzyme APOBEC-1",
  "gene_symbol": "APOBEC1",
  "term_label": "cytidine deaminase activity",
  "gene": "UniProtKB:P41238"
}